{
  "term_label": "mitochondrial calcium ion homeostasis",
  "term_id": "GO:0051560",
  "gene_symbol": "MCU",
  "gene": "UniProtKB:Q8NE86",
  "gene_name": "Calcium uniporter protein, mitochondrial"
}